{
  "gene_name": "Nucleolar protein 10",
  "term_id": "GO:0005730",
  "gene_symbol": "NOL10",
  "term_label": "nucleolus",
  "gene": "UniProtKB:Q9BSC4"
}